mannitol 2-dehydrogenase activity [GO:0050086] (molecular function) Definition: Catalysis of the reaction: D-mannitol + NAD+ = D-fructose + NADH. Sources: EC:1.1.1.67, MetaCyc:MANNITOL-2-DEHYDROGENASE-RXN Relationships: is a type of oxidoreductase activity, acting on the CH-OH group of donors, NAD or NADP as acceptor [GO:0016616] Also known as: D-mannitol dehydrogenase activity, D-mannitol:NAD+ 2-oxidoreductase activity